{
  "gene_symbol": "RBP7",
  "gene_name": "Retinoid-binding protein 7",
  "gene": "UniProtKB:Q96R05",
  "term_label": "fatty acid transport",
  "term_id": "GO:0015908"
}